maintenance of synapse structure [GO:0099558] (BP) References: PMID:24449494, PMID:25611509 Sources: GOC:dos Relationships: is a type of cell junction maintenance [GO:0034331]; is a type of synapse organization [GO:0050808] Definition: A process that preserves the structural organistation and orientation of a synaptic cellular component such as the synaptic cytoskeleton and molecular scaffolds. Also known as: synaptic maintenance Subtypes: maintenance of presynaptic active zone structure [GO:0048790], GO:0098880, GO:0099559